positive regulation of protein localization to cell surface [GO:2000010] (BP) Also known as: positive regulation of protein localisation at cell surface, positive regulation of protein localization at cell surface Definition: Any process that activates or increases the frequency, rate or extent of protein localization to the cell surface. Relationships: is a type of GO:1903829; is a type of regulation of protein localization to cell surface [GO:2000008]; positively regulates protein localization to cell surface [GO:0034394] Sources: GOC:obol